{
  "gene_symbol": "NDUFV3",
  "term_id": "GO:0045271",
  "gene_name": "NADH dehydrogenase [ubiquinone] flavoprotein 3, mitochondrial",
  "term_label": "respiratory chain complex I",
  "gene": "UniProtKB:P56181"
}